{
  "gene_symbol": "GKN2",
  "term_label": "regulation of cell population proliferation",
  "term_id": "GO:0042127",
  "gene": "UniProtKB:Q86XP6",
  "gene_name": "Gastrokine-2"
}